{
  "gene": "UniProtKB:Q6IS14",
  "gene_name": "Eukaryotic translation initiation factor 5A-1-like",
  "gene_symbol": "EIF5AL1",
  "term_id": "GO:0003746",
  "term_label": "translation elongation factor activity"
}